{
  "gene_name": "Disheveled-associated activator of morphogenesis 2",
  "term_label": "regulation of non-canonical Wnt signaling pathway",
  "gene_symbol": "DAAM2",
  "term_id": "GO:2000050",
  "gene": "UniProtKB:Q86T65"
}